{
  "gene_name": "Vasopressin-neurophysin 2-copeptin",
  "term_label": "extracellular space",
  "gene": "UniProtKB:P01185",
  "term_id": "GO:0005615",
  "gene_symbol": "AVP"
}